{
  "gene_symbol": "SPTA1",
  "gene": "UniProtKB:P02549",
  "term_id": "GO:0042995",
  "gene_name": "Spectrin alpha chain, erythrocytic 1",
  "term_label": "cell projection"
}